proton motive force-driven mitochondrial ATP synthesis [GO:0042776] (biological process) Definition: The chemical reactions and pathways resulting in the formation of ATP driven by transport of protons across a mitochondrial membrane to generate an electrochemical gradient (proton-motive force). Sources: GOC:vw Also known as: mitochondrial ATP synthesis coupled proton transport, mitochondrial proton transport Relationships: is a type of proton motive force-driven ATP synthesis [GO:0015986]; is part of oxidative phosphorylation [GO:0006119]; occurs in GO:0005739 Regulation: regulated by regulation of mitochondrial ATP synthesis coupled proton transport [GO:1905706]; negatively regulated by negative regulation of mitochondrial ATP synthesis coupled proton transport [GO:1905707]